{
  "gene_symbol": "SLC25A12",
  "gene": "UniProtKB:O75746",
  "term_label": "L-glutamate transmembrane transporter activity",
  "gene_name": "Electrogenic aspartate_glutamate antiporter SLC25A12, mitochondrial",
  "term_id": "GO:0005313"
}